negative regulation of protein localization to Cajal body [GO:1904870] (biological process) Definition: Any process that stops, prevents or reduces the frequency, rate or extent of protein localization to Cajal body. Relationships: is a type of negative regulation of protein localization to nucleus [GO:1900181]; is a type of regulation of protein localization to Cajal body [GO:1904869]; negatively regulates protein localization to Cajal body [GO:1904867] Also known as: down regulation of protein localisation in Cajal body, down regulation of protein localisation to Cajal body, down regulation of protein localization in Cajal body, down regulation of protein localization to Cajal body, down-regulation of protein localisation in Cajal body, down-regulation of protein localisation to Cajal body, down-regulation of protein localization in Cajal body, down-regulation of protein localization to Cajal body, downregulation of protein localisation in Cajal body, downregulation of protein localisation to Cajal body, downregulation of protein localization in Cajal body, downregulation of protein localization to Cajal body, negative regulation of protein localisation in Cajal body, negative regulation of protein localisation to Cajal body, negative regulation of protein localization in Cajal body, inhibition of protein localisation in Cajal body, inhibition of protein localisation to Cajal body, inhibition of protein localization in Cajal body, inhibition of protein localization to Cajal body References: PMID:25467444 Sources: GOC:BHF, GOC:BHF_telomere, GOC:TermGenie, GOC:nc, GO_REF:0000058